{
  "gene": "UniProtKB:Q15059",
  "term_label": "nucleus",
  "gene_name": "Bromodomain-containing protein 3",
  "gene_symbol": "BRD3",
  "term_id": "GO:0005634"
}